{
  "term_id": "GO:0010758",
  "gene": "UniProtKB:Q9ULD2",
  "gene_name": "Microtubule-associated tumor suppressor 1",
  "gene_symbol": "MTUS1",
  "term_label": "regulation of macrophage chemotaxis"
}